{
  "term_label": "Unknown molecular function",
  "gene_symbol": "IKBKE-AS1",
  "term_id": "UNKNOWN:0001",
  "gene_name": "Putative uncharacterized protein IKBKE-AS1",
  "gene": "UniProtKB:Q96MC9"
}